{
  "gene_name": "Conserved oligomeric Golgi complex subunit 4",
  "gene": "UniProtKB:Q9H9E3",
  "term_label": "retrograde vesicle-mediated transport, Golgi to endoplasmic reticulum",
  "term_id": "GO:0006890",
  "gene_symbol": "COG4"
}